stress response to nickel ion [GO:1990532] (biological process) Definition: Any process that results in a change in state or activity of a cell or an organism (in terms of movement, secretion, enzyme production, gene expression, etc.) as a result of a disturbance in organismal or cellular homeostasis caused by a nickel ion stimulus. References: PMID:25330323 Sources: GOC:kmv Also known as: response to nickel ion stress, response to nickel toxicity, stress response to nickel Relationships: is a type of stress response to metal ion [GO:0097501]